{
  "term_id": "GO:0000978",
  "gene_name": "Zinc finger protein with KRAB and SCAN domains 4",
  "gene": "UniProtKB:Q969J2",
  "term_label": "RNA polymerase II cis-regulatory region sequence-specific DNA binding",
  "gene_symbol": "ZKSCAN4"
}